{
  "gene": "UniProtKB:Q9BR39",
  "gene_name": "Junctophilin-2",
  "term_id": "UNKNOWN:0001",
  "gene_symbol": "JPH2",
  "term_label": "Unknown molecular function"
}